{
  "gene": "UniProtKB:Q8TBB0",
  "gene_name": "THAP domain-containing protein 6",
  "term_id": "UNKNOWN:0001",
  "term_label": "Unknown molecular function",
  "gene_symbol": "THAP6"
}